{
  "term_id": "GO:0045944",
  "gene_symbol": "NEUROG1",
  "gene": "UniProtKB:Q92886",
  "term_label": "positive regulation of transcription by RNA polymerase II",
  "gene_name": "Neurogenin-1"
}